{
  "term_label": "RNA polymerase II cis-regulatory region sequence-specific DNA binding",
  "term_id": "GO:0000978",
  "gene_name": "Zinc finger protein 449",
  "gene": "UniProtKB:Q6P9G9",
  "gene_symbol": "ZNF449"
}